{
  "term_label": "extracellular space",
  "term_id": "GO:0005615",
  "gene_name": "Tenascin-R",
  "gene_symbol": "TNR",
  "gene": "UniProtKB:Q92752"
}